{
  "gene": "UniProtKB:P29274",
  "gene_symbol": "ADORA2A",
  "term_label": "plasma membrane",
  "term_id": "GO:0005886",
  "gene_name": "Adenosine receptor A2a"
}